{
  "gene": "UniProtKB:P16109",
  "gene_name": "P-selectin",
  "term_label": "sialic acid binding",
  "gene_symbol": "SELP",
  "term_id": "GO:0033691"
}